{
  "gene": "UniProtKB:P22674",
  "term_id": "GO:0016538",
  "gene_name": "Cyclin-O",
  "gene_symbol": "CCNO",
  "term_label": "cyclin-dependent protein serine/threonine kinase regulator activity"
}